{
  "gene_name": "Fc receptor-like protein 3",
  "term_id": "GO:0006955",
  "gene": "UniProtKB:Q96P31",
  "gene_symbol": "FCRL3",
  "term_label": "immune response"
}